{
  "gene_symbol": "FAM120B",
  "gene_name": "Constitutive coactivator of peroxisome proliferator-activated receptor gamma",
  "term_id": "UNKNOWN:0001",
  "gene": "UniProtKB:Q96EK7",
  "term_label": "Unknown molecular function"
}